{
  "gene_symbol": "ADIPOQ",
  "term_id": "UNKNOWN:0001",
  "term_label": "Unknown molecular function",
  "gene_name": "Adiponectin",
  "gene": "UniProtKB:Q15848"
}